{
  "gene": "UniProtKB:P12755",
  "term_id": "GO:0005737",
  "gene_name": "Ski oncogene",
  "term_label": "cytoplasm",
  "gene_symbol": "SKI"
}